copalyl diphosphate synthase activity [GO:0050559] (molecular function) Definition: Catalysis of the reaction: all-trans-geranylgeranyl diphosphate = (+)-copalyl diphosphate. Sources: EC:5.5.1.12, RHEA:24316 Relationships: is a type of intramolecular lyase activity [GO:0016872] Also known as: diterpene cyclase activity, (+)-copalyl-diphosphate lyase (decyclizing)